negative regulation of cytokine-mediated signaling pathway [GO:0001960] (biological process) Also known as: down regulation of cytokine mediated signaling pathway, down-regulation of cytokine mediated signaling pathway, downregulation of cytokine mediated signaling pathway, negative regulation of cytokine and chemokine mediated signaling pathway, negative regulation of cytokine mediated signaling pathway, negative regulation of cytokine mediated signalling pathway, inhibition of cytokine mediated signaling pathway Definition: Any process that stops, prevents, or reduces the frequency, rate or extent of the cytokine mediated signaling pathway. Sources: GOC:hjd Subtypes: negative regulation of tumor necrosis factor-mediated signaling pathway [GO:0010804], GO:0060336, GO:0060339, negative regulation of chemokine-mediated signaling pathway [GO:0070100], negative regulation of interleukin-6-mediated signaling pathway [GO:0070104], negative regulation of interleukin-27-mediated signaling pathway [GO:0070108], GO:0070759, GO:1900235, negative regulation of interleukin-2-mediated signaling pathway [GO:1902206], negative regulation of prolactin signaling pathway [GO:1902212], negative regulation of interleukin-4-mediated signaling pathway [GO:1902215], negative regulation of macrophage colony-stimulating factor signaling pathway [GO:1902227], negative regulation of interleukin-17-mediated signaling pathway [GO:1903882], negative regulation of macrophage migration inhibitory factor signaling pathway [GO:2000447], negative regulation of interleukin-18-mediated signaling pathway [GO:2000493], negative regulation of interleukin-1-mediated signaling pathway [GO:2000660] Relationships: is a type of GO:0001959; is a type of negative regulation of signal transduction [GO:0009968]; is a type of negative regulation of response to cytokine stimulus [GO:0060761]; negatively regulates cytokine-mediated signaling pathway [GO:0019221]